{
  "gene_name": "Arylsulfatase K",
  "gene": "UniProtKB:Q6UWY0",
  "gene_symbol": "ARSK",
  "term_id": "UNKNOWN:0003",
  "term_label": "Unknown cellular component"
}